{
  "gene_name": "Beta-actin-like protein 2",
  "term_label": "cell motility",
  "gene": "UniProtKB:Q562R1",
  "gene_symbol": "ACTBL2",
  "term_id": "GO:0048870"
}